{
  "gene_name": "ADP-ribosylation factor 3",
  "gene_symbol": "ARF3",
  "gene": "UniProtKB:P61204",
  "term_id": "GO:0005525",
  "term_label": "GTP binding"
}